embryonic morphogenesis [GO:0048598] (biological process) Definition: The process in which anatomical structures are generated and organized during the embryonic phase. The embryonic phase begins with zygote formation. The end of the embryonic phase is organism-specific. For example, it would be at birth for mammals, larval hatching for insects and seed dormancy in plants. Sources: GOC:jid, GOC:mtg_sensu Relationships: is a type of GO:0009653; is part of embryo development [GO:0009790] Also known as: embryonic anatomical structure morphogenesis Subtypes: inner cell mass cellular morphogenesis [GO:0001828], trophectodermal cellular morphogenesis [GO:0001831], GO:0002093, embryonic heart tube morphogenesis [GO:0003143], GO:0003152, heart rudiment morphogenesis [GO:0003314], pericardium morphogenesis [GO:0003344], optic vesicle morphogenesis [GO:0003404], GO:0007369, GO:0007374, GO:0007377, germ-band shortening [GO:0007390], GO:0007392, GO:0007394, GO:0007396, Malpighian tubule morphogenesis [GO:0007443], head involution [GO:0008258], embryonic shoot morphogenesis [GO:0010064], embryonic root morphogenesis [GO:0010086], GO:0010172, neural plate elongation [GO:0014022], morphogenesis of embryonic epithelium [GO:0016331], neural fold bending [GO:0021503], GO:0021505, midbrain-hindbrain boundary morphogenesis [GO:0021555], GO:0021991, GO:0021993, GO:0032474, GO:0033505, embryonic appendage morphogenesis [GO:0035113], embryonic nail plate morphogenesis [GO:0035880], inner ear morphogenesis [GO:0042472], GO:0042473, middle ear morphogenesis [GO:0042474], GO:0042733, GO:0046664, embryo sac morphogenesis [GO:0048314], embryonic organ morphogenesis [GO:0048562], embryonic ectodermal digestive tract morphogenesis [GO:0048613], GO:0048617, GO:0048619, embryonic neurocranium morphogenesis [GO:0048702], embryonic viscerocranium morphogenesis [GO:0048703], semicircular canal morphogenesis [GO:0048752], GO:0048826, invagination involved in gastrulation with mouth forming second [GO:0055109], involution involved in gastrulation with mouth forming second [GO:0055110], GO:0055113, convergent extension involved in gastrulation [GO:0060027], GO:0060059, vestibular receptor cell morphogenesis [GO:0060116], embryonic placenta morphogenesis [GO:0060669], branching involved in labyrinthine layer morphogenesis [GO:0060670], epithelial cell morphogenesis involved in placental branching [GO:0060672], labyrinthine layer morphogenesis [GO:0060713], mesodermal to mesenchymal transition involved in gastrulation [GO:0060809], pouch outgrowth involved in semicircular canal formation [GO:0060878], cell morphogenesis involved in semicircular canal fusion [GO:0060880], clearance of cells from fusion plate [GO:0060884], olfactory placode morphogenesis [GO:0071699], zygote elongation [GO:0080159], cochlea morphogenesis [GO:0090103], establishment of planar polarity involved in neural tube closure [GO:0090177]